{
  "gene": "UniProtKB:O95388",
  "term_id": "GO:0007155",
  "term_label": "cell adhesion",
  "gene_name": "CCN family member 4",
  "gene_symbol": "CCN4"
}